{
  "term_id": "UNKNOWN:0001",
  "gene_symbol": "FAM47DP",
  "gene": "UniProtKB:A6NHR8",
  "term_label": "Unknown molecular function",
  "gene_name": "Putative protein FAM47D"
}